amylin binding [GO:0097645] (molecular function) Definition: Binding to amylin. References: PMID:10871296, PMID:12037140, PMID:18687416 Sources: GOC:bhm Relationships: is a type of calcitonin family binding [GO:0097644]